{
  "gene": "UniProtKB:P62829",
  "gene_name": "Large ribosomal subunit protein uL14",
  "term_id": "GO:0070180",
  "term_label": "large ribosomal subunit rRNA binding",
  "gene_symbol": "RPL23"
}